{
  "gene": "UniProtKB:Q8N3C7",
  "term_id": "GO:0005634",
  "term_label": "nucleus",
  "gene_name": "CAP-Gly domain-containing linker protein 4",
  "gene_symbol": "CLIP4"
}